calcium-induced calcium release activity involved in regulation of presynaptic cytosolic calcium ion concentration [GO:1905054] (molecular function) References: PMID:15919193, PMID:23918386 Sources: GOC:TermGenie, GO_REF:0000061 Relationships: is a type of calcium-induced calcium release activity [GO:0048763]; is part of GO:0099509 Also known as: calcium-induced calcium release activity involved in regulation of presynaptic cytosolic calcium levels Definition: Any calcium-induced calcium release activity that is involved in regulation of presynaptic cytosolic calcium ion concentration.